{
  "term_label": "vesicle docking involved in exocytosis",
  "gene_symbol": "VPS18",
  "gene": "UniProtKB:Q9P253",
  "term_id": "GO:0006904",
  "gene_name": "Vacuolar protein sorting-associated protein 18 homolog"
}